epidermal growth factor receptor signaling pathway [GO:0007173] (biological process) Regulation: regulated by regulation of epidermal growth factor receptor signaling pathway [GO:0042058]; negatively regulated by GO:0042059; positively regulated by positive regulation of epidermal growth factor receptor signaling pathway [GO:0045742] Also known as: EGF receptor signaling pathway, EGF receptor signalling pathway, EGFR signaling pathway, ERBB1 signaling pathway, epidermal growth factor receptor signalling pathway, receptor tyrosine-protein kinase erbB-1 signaling pathway Subtypes: epidermal growth factor signaling pathway involved in forebrain neuron fate commitment [GO:0022026], ERBB2-EGFR signaling pathway [GO:0038134], ERBB4-EGFR signaling pathway [GO:0038137], epidermal growth factor receptor signaling pathway involved in lung development [GO:0060507], epidermal growth factor receptor signaling pathway involved in heart process [GO:1905251] Relationships: is a type of GO:0038127 Sources: GOC:ceb Definition: The series of molecular signals initiated by binding of a ligand to the tyrosine kinase receptor EGFR (ERBB1) on the surface of a cell. The pathway ends with regulation of a downstream cellular process, e.g. transcription.